natural killer cell inhibitory signaling pathway [GO:0002769] (biological process) Definition: The series of molecular signals initiated by an extracellular ligand binding to a receptor on the surface of a natural killer cell capable of inhibiting an immune effector process contributing to an immune response. References: PMID:15771571 Sources: GOC:add, ISBN:0781735149 Also known as: NK cell inhibitory signaling pathway, natural killer cell inhibitory signalling pathway, inhibitory KIR signaling pathway, killer cell inhibitory receptor signaling pathway, Ly49 inhibitory receptor signaling pathway Relationships: is a type of GO:0002767